{
  "gene_symbol": "SH3GL3",
  "term_label": "membrane",
  "gene": "UniProtKB:Q99963",
  "term_id": "GO:0016020",
  "gene_name": "Endophilin-A3"
}